{
  "term_label": "GID complex",
  "gene_symbol": "WDR26",
  "gene_name": "WD repeat-containing protein 26",
  "term_id": "GO:0034657",
  "gene": "UniProtKB:Q9H7D7"
}